{
  "gene": "UniProtKB:Q5VWP2",
  "gene_name": "Terminal nucleotidyltransferase 5C",
  "term_id": "UNKNOWN:0003",
  "gene_symbol": "TENT5C",
  "term_label": "Unknown cellular component"
}